{
  "gene": "UniProtKB:Q9Y587",
  "term_label": "Unknown cellular component",
  "gene_name": "AP-4 complex subunit sigma-1",
  "term_id": "UNKNOWN:0003",
  "gene_symbol": "AP4S1"
}